{
  "gene_symbol": "DCAF1",
  "gene": "UniProtKB:Q9Y4B6",
  "term_label": "nucleus",
  "term_id": "GO:0005634",
  "gene_name": "DDB1- and CUL4-associated factor 1"
}